{
  "gene": "UniProtKB:O15169",
  "gene_name": "Axin-1",
  "gene_symbol": "AXIN1",
  "term_id": "GO:0042802",
  "term_label": "identical protein binding"
}